{
  "gene": "UniProtKB:Q9NVR5",
  "gene_name": "Protein kintoun",
  "term_label": "axonemal dynein complex assembly",
  "gene_symbol": "DNAAF2",
  "term_id": "GO:0070286"
}